{
  "gene": "UniProtKB:Q9C0J9",
  "gene_name": "Class E basic helix-loop-helix protein 41",
  "term_label": "DNA-binding transcription factor activity, RNA polymerase II-specific",
  "term_id": "GO:0000981",
  "gene_symbol": "BHLHE41"
}